{
  "gene": "UniProtKB:Q68CZ6",
  "term_id": "GO:0072686",
  "term_label": "mitotic spindle",
  "gene_symbol": "HAUS3",
  "gene_name": "HAUS augmin-like complex subunit 3"
}